{
  "term_id": "GO:0006974",
  "gene": "UniProtKB:Q9Y3S1",
  "gene_name": "Serine_threonine-protein kinase WNK2",
  "gene_symbol": "WNK2",
  "term_label": "DNA damage response"
}